interleukin-23 production [GO:0032627] (biological process) Relationships: is a type of GO:0001816 Definition: The appearance of interleukin-23 due to biosynthesis or secretion following a cellular stimulus, resulting in an increase in its intracellular or extracellular levels. Also known as: IL-23 production, interleukin-23 biosynthetic process, interleukin-23 secretion Regulation: regulated by regulation of interleukin-23 production [GO:0032667]; RO_0002212 by GO:0032707; positively regulated by positive regulation of interleukin-23 production [GO:0032747] Sources: GOC:mah